{
  "gene": "UniProtKB:P0CG04",
  "gene_name": "Immunoglobulin lambda constant 1",
  "gene_symbol": "IGLC1",
  "term_label": "antigen binding",
  "term_id": "GO:0003823"
}